positive regulation of infection cushion formation [GO:0075185] (biological process) Relationships: is a type of positive regulation of developmental process [GO:0051094]; is a type of regulation of infection cushion formation [GO:0075184]; positively regulates infection cushion formation [GO:0075183] Also known as: positive regulation of infection cushion formation on or near host Definition: Any process that activates or increases the frequency, rate or extent of symbiont infection cushion formation on or near its host organism. The host is defined as the larger of the organisms involved in a symbiotic interaction. Sources: GOC:pamgo_curators